{
  "gene_name": "Sodium channel protein type 2 subunit alpha",
  "gene": "UniProtKB:Q99250",
  "term_id": "GO:0005248",
  "gene_symbol": "SCN2A",
  "term_label": "voltage-gated sodium channel activity"
}